structural constituent of adult chitin-based cuticle [GO:0008012] (molecular function) Relationships: is a type of GO:0005214 Sources: GOC:mah, GOC:mtg_sensu Also known as: structural constituent of adult cuticle Definition: The action of a molecule that contributes to the structural integrity of the chitin-based cuticle of an adult organism. An example of this is found in Drosophila melanogaster.